glucokinase activity [GO:0004340] (MF) Regulation: negatively regulated by negative regulation of glucokinase activity [GO:0033132] Also known as: ATP:D-glucose 6-phosphotransferase activity, glucokinase (phosphorylating), glucose kinase activity Relationships: is a type of hexokinase activity [GO:0004396]; is part of GO:0051156 Definition: Catalysis of the reaction: ATP + D-glucose = ADP + D-glucose-6-phosphate. Sources: EC:2.7.1.2